{
  "gene_symbol": "CARMIL3",
  "gene_name": "Capping protein, Arp2_3 and myosin-I linker protein 3",
  "gene": "UniProtKB:Q8ND23",
  "term_label": "Unknown molecular function",
  "term_id": "UNKNOWN:0001"
}